{
  "gene": "UniProtKB:Q9UQF2",
  "gene_symbol": "MAPK8IP1",
  "term_label": "MAP-kinase scaffold activity",
  "gene_name": "C-Jun-amino-terminal kinase-interacting protein 1",
  "term_id": "GO:0005078"
}